{
  "gene_symbol": "NTHL1",
  "gene": "UniProtKB:P78549",
  "gene_name": "Endonuclease III-like protein 1",
  "term_id": "GO:0006285",
  "term_label": "base-excision repair, AP site formation"
}